{
  "gene_name": "[F-actin]-monooxygenase MICAL2",
  "gene": "UniProtKB:O94851",
  "term_id": "GO:0003779",
  "gene_symbol": "MICAL2",
  "term_label": "actin binding"
}